{
  "gene_symbol": "PAX3",
  "term_id": "GO:0007399",
  "term_label": "nervous system development",
  "gene_name": "Paired box protein Pax-3",
  "gene": "UniProtKB:P23760"
}